{
  "term_label": "proteasome-mediated ubiquitin-dependent protein catabolic process",
  "term_id": "GO:0043161",
  "gene": "UniProtKB:P68543",
  "gene_name": "UBX domain-containing protein 2A",
  "gene_symbol": "UBXN2A"
}